dehydroepiandrosterone secretion [GO:0035942] (biological process) Regulation: regulated by regulation of dehydroepiandrosterone secretion [GO:2000840]; negatively regulated by negative regulation of dehydroepiandrosterone secretion [GO:2000841]; RO_0002213 by GO:2000842 Relationships: is a type of organic hydroxy compound transport [GO:0015850]; is a type of hormone secretion [GO:0046879]; is a type of lipid export from cell [GO:0140353] Also known as: 3beta-hydroxyandrost-5-en-17-one secretion, DHEA secretion, dehydroisoandrosterone secretion Definition: The regulated release of dehydroepiandrosterone (3beta-hydroxyandrost-5-en-17-one) into the circulatory system. Sources: GOC:sl